{
  "gene_symbol": "TMEM78",
  "gene": "UniProtKB:Q5T7P6",
  "term_label": "Unknown biological process",
  "term_id": "UNKNOWN:0002",
  "gene_name": "Transmembrane protein 78"
}